{
  "gene_name": "Ribosome maturation protein SBDS",
  "term_label": "Unknown cellular component",
  "gene_symbol": "SBDS",
  "term_id": "UNKNOWN:0003",
  "gene": "UniProtKB:Q9Y3A5"
}